{
  "term_label": "heart development",
  "gene_name": "Histone demethylase UTY",
  "gene": "UniProtKB:O14607",
  "gene_symbol": "UTY",
  "term_id": "GO:0007507"
}